{
  "gene_symbol": "CTU2",
  "gene_name": "Cytoplasmic tRNA 2-thiolation protein 2",
  "term_id": "GO:0005829",
  "term_label": "cytosol",
  "gene": "UniProtKB:Q2VPK5"
}